{
  "gene_symbol": "ABLIM1",
  "term_id": "GO:0060271",
  "gene_name": "Actin-binding LIM protein 1",
  "term_label": "cilium assembly",
  "gene": "UniProtKB:O14639"
}